{
  "gene_symbol": "NR1D1",
  "gene": "UniProtKB:P20393",
  "gene_name": "Nuclear receptor subfamily 1 group D member 1",
  "term_label": "hormone-mediated signaling pathway",
  "term_id": "GO:0009755"
}